germarium-derived oocyte differentiation [GO:0030706] (biological process) Also known as: oocyte cell differentiation Relationships: is a type of oocyte differentiation [GO:0009994]; is part of germarium-derived egg chamber formation [GO:0007293] Definition: The process in which one relatively unspecialized immature cystocyte of the germ-line cyst in the germarium acquires the specialized features of an oocyte. An example of this process can be found in Drosophila melanogaster. Sources: GOC:mtg_sensu, ISBN:0879694238